calcium-dependent cysteine-type endopeptidase activity [GO:0004198] (molecular function) Relationships: is a type of cysteine-type endopeptidase activity [GO:0004197] Sources: GOC:mah Also known as: calpain activity Definition: Catalysis of the hydrolysis of nonterminal peptide bonds in a polypeptide chain by a mechanism using a cysteine residue at the enzyme active center, and requiring the presence of calcium.